response to undecane [GO:1902784] (biological process) Relationships: is_a response to alkane [GO:1902778] Subtypes: cellular response to undecane [GO:1902785] Definition: Any process that results in a change in state or activity of a cell or an organism (in terms of movement, secretion, enzyme production, gene expression, etc.) as a result of an undecane stimulus. References: PMID:23826995 Sources: GOC:TermGenie, GOC:mengo_curators, GO_REF:0000071